purine ribonucleotide binding [GO:0032555] (molecular function) Definition: Binding to a purine ribonucleotide, any compound consisting of a purine ribonucleoside that is esterified with (ortho)phosphate or an oligophosphate at any hydroxyl group on the ribose moiety. Sources: GOC:mah Relationships: is a type of purine nucleotide binding [GO:0017076]; is a type of ribonucleotide binding [GO:0032553] Subtypes: GO:0032559, guanyl ribonucleotide binding [GO:0032561], XTP binding [GO:1901640], ITP binding [GO:1901641], IMP binding [GO:1902249]